{
  "term_id": "GO:0019731",
  "term_label": "antibacterial humoral response",
  "gene_symbol": "IGHA1",
  "gene": "UniProtKB:P01876",
  "gene_name": "Immunoglobulin heavy constant alpha 1"
}